{
  "gene_symbol": "MCTS1",
  "term_id": "UNKNOWN:0003",
  "gene": "UniProtKB:Q9ULC4",
  "term_label": "Unknown cellular component",
  "gene_name": "Malignant T-cell-amplified sequence 1"
}